{
  "gene_symbol": "MYLK3",
  "gene": "UniProtKB:Q32MK0",
  "term_label": "signal transduction",
  "gene_name": "Myosin light chain kinase 3",
  "term_id": "GO:0007165"
}